{
  "gene": "UniProtKB:Q8NDW8",
  "term_id": "GO:0030991",
  "term_label": "intraciliary transport particle A",
  "gene_name": "Tetratricopeptide repeat protein 21A",
  "gene_symbol": "TTC21A"
}